neurotransmitter secretion [GO:0007269] (biological process) Regulation: positively regulated by positive regulation of neurotransmitter secretion [GO:0001956]; regulated by GO:0046928; negatively regulated by negative regulation of neurotransmitter secretion [GO:0046929] Subtypes: acetylcholine secretion, neurotransmission [GO:0014055], neurotransmitter secretion involved in regulation of skeletal muscle contraction [GO:0014860], spontaneous exocytosis of neurotransmitter [GO:0048792], serotonin secretion, neurotransmission [GO:0060096], GO:0061530, primary amine secretion, neurotransmission [GO:0061532], gamma-aminobutyric acid secretion, neurotransmission [GO:0061534], GO:0061535, glycine secretion, neurotransmission [GO:0061537], GO:0061538, octopamine secretion, neurotransmission [GO:0061540], GO:0061544, GO:0061669, evoked neurotransmitter secretion [GO:0061670], synchronous neurotransmitter secretion [GO:0071911], asynchronous neurotransmitter secretion [GO:0071912], GO:0160043, GO:1990793 Relationships: is a type of neurotransmitter transport [GO:0006836]; is a type of establishment of localization in cell [GO:0051649]; is a type of signal release from synapse [GO:0099643]; is part of chemical synaptic transmission [GO:0007268]; occurs in presynapse [GO:0098793] Sources: GOC:dph Note: A neurotransmitter is any of a group of substances that are released on excitation from the axon terminal of a presynaptic neuron of the central or peripheral nervous system and travel across the synaptic cleft to either excite or inhibit the target cell. Among the many substances that have the properties of a neurotransmitter are acetylcholine, noradrenaline, adrenaline, dopamine, glycine, gamma-aminobutyrate, glutamic acid, substance P, enkephalins, endorphins and serotonin. Definition: The regulated release of neurotransmitter from the presynapse into the synaptic cleft via calcium-regulated exocytosis during synaptic transmission. Also known as: neurotransmitter release, neurotransmitter secretory pathway